{
  "term_label": "trans-Golgi network",
  "term_id": "GO:0005802",
  "gene": "UniProtKB:O43493",
  "gene_symbol": "TGOLN2",
  "gene_name": "Trans-Golgi network integral membrane protein 2"
}